negative regulation of nodal receptor complex assembly [GO:1900124] (biological process) References: PMID:15062104 Sources: GOC:TermGenie, GOC:signaling Definition: Any process that stops, prevents or reduces the frequency, rate or extent of nodal receptor complex assembly. Also known as: down regulation of ActRIIB.ALK4.EGF-CFC complex formation, down regulation of nodal receptor complex assembly, down regulation of nodal receptor complex formation, down-regulation of ActRIIB.ALK4.EGF-CFC complex formation, down-regulation of nodal receptor complex assembly, down-regulation of nodal receptor complex formation, downregulation of ActRIIB.ALK4.EGF-CFC complex formation, downregulation of nodal receptor complex assembly, downregulation of nodal receptor complex formation, negative regulation of ActRIIB.ALK4.EGF-CFC complex formation, negative regulation of nodal receptor complex formation, inhibition of ActRIIB.ALK4.EGF-CFC complex formation, inhibition of nodal receptor complex assembly, inhibition of nodal receptor complex formation Relationships: is a type of negative regulation of protein-containing complex assembly [GO:0031333]; is a type of regulation of nodal receptor complex assembly [GO:1900123]; negatively regulates nodal receptor complex assembly [GO:0038099]